{
  "gene_name": "Zinc finger protein 610",
  "gene": "UniProtKB:Q8N9Z0",
  "term_id": "GO:0000981",
  "term_label": "DNA-binding transcription factor activity, RNA polymerase II-specific",
  "gene_symbol": "ZNF610"
}